{
  "gene_symbol": "SAGE2P",
  "term_id": "GO:0032039",
  "gene": "UniProtKB:A6NJ88",
  "gene_name": "Putative SAGE1-like protein",
  "term_label": "integrator complex"
}